FtsBL complex [GO:1990588] (cellular component) Definition: A protein complex required for prokaryotic cell division (FtsZ-dependent cytokinesis). Part of the divisome. Assembled independently of the other divisome components in the cytoplasm prior to transport to the cell septum. In E. coli consists of FtsB and FtsL. Note: An example of this is FtsB in E. coli (P0A6S5) in PMID:15165235 (inferred from physical interaction). Relationships: is a type of divisome complex [GO:1990586]; is part of GO:0005829; is part of GO:1990587 References: PMID:15165235, PMID:21784946 Sources: GOC:bhm Also known as: FtsB-FtsL complex